{
  "gene_symbol": "STK26",
  "gene_name": "Serine_threonine-protein kinase 26",
  "term_label": "negative regulation of cell migration",
  "term_id": "GO:0030336",
  "gene": "UniProtKB:Q9P289"
}